regulation of zinc ion transport [GO:0071579] (BP) Definition: Any process that modulates the frequency, rate or extent of the directed movement of zinc ions (Zn2+) into, out of or within a cell, or between cells, by means of some agent such as a transporter or pore. Sources: GOC:BHF, GOC:mah Relationships: is a type of GO:0010959; regulates zinc ion transport [GO:0006829] Subtypes: regulation of zinc ion transmembrane transport [GO:0071580], GO:0071582